{
  "gene": "UniProtKB:Q96CD2",
  "gene_symbol": "PPCDC",
  "gene_name": "Phosphopantothenoylcysteine decarboxylase",
  "term_id": "GO:0010181",
  "term_label": "FMN binding"
}